glutamatergic postsynaptic density [GO:0099573] (cellular component) Also known as: postsynaptic specialization, glutamatergic neuron-to-neuron synapse Relationships: is a type of GO:0014069 Sources: GOC:dos Definition: The post-synaptic specialization of a glutamatergic excitatory synapse.